{
  "gene": "UniProtKB:P10415",
  "term_id": "GO:0043065",
  "term_label": "positive regulation of apoptotic process",
  "gene_symbol": "BCL2",
  "gene_name": "Apoptosis regulator Bcl-2"
}